positive regulation of torso signaling pathway [GO:0120176] (biological process) References: PMID:23732470 Sources: GOC:ha Relationships: is a type of positive regulation of signal transduction [GO:0009967]; is a type of GO:0120175; positively regulates torso signaling pathway [GO:0008293] Definition: Any process that activates or increases the frequency, rate or extent of the torso signaling pathway.